{
  "gene": "UniProtKB:Q5BKY1",
  "gene_name": "Leucine-rich repeat-containing protein 10",
  "gene_symbol": "LRRC10",
  "term_label": "cytoskeleton",
  "term_id": "GO:0005856"
}